anthocyanin 5-O-glucoside 6'''-O-malonyltransferase activity [GO:0033810] (molecular function) Relationships: is a type of acyltransferase activity, transferring groups other than amino-acyl groups [GO:0016747] Sources: EC:2.3.1.172 Also known as: Ss5MaT1, malonyl-CoA:pelargonidin-3-O-(6-caffeoyl-beta-D-glucoside)-5-O-beta-D-glucoside 6'''-O-malonyltransferase activity Definition: Catalysis of the reaction: malonyl-CoA + pelargonidin 3-O-(6-caffeoyl-beta-D-glucoside) 5-O-beta-D-glucoside = CoA + 4'''-demalonylsalvianin.